stereocilium [GO:0032420] (cellular component) Definition: An actin-based protrusion from the apical surface of auditory and vestibular hair cells and of neuromast cells. These protrusions are supported by a bundle of cross-linked actin filaments (an actin cable), oriented such that the plus (barbed) ends are at the tip of the protrusion, capped by a tip complex which bridges to the plasma. Bundles of stereocilia act as mechanosensory organelles. References: PMID:15661519, PMID:7840137 Sources: GOC:ecd Relationships: is a type of neuron projection [GO:0043005]; is a type of actin-based cell projection [GO:0098858]; is part of stereocilium bundle [GO:0032421]; is part of organelle [GO:0043226]